thalianol synthase activity [GO:0051746] (molecular function) References: PMID:15125655 Sources: RHEA:26160 Definition: Catalysis of the cyclization of 3(S)-oxidosqualene to (3S,13S,14R)-malabarica-8,17,21-trien-3-ol (thalianol). Relationships: is a type of oxidosqualene cyclase activity [GO:0031559]